{
  "gene_symbol": "LTB4R",
  "term_id": "GO:0008528",
  "gene": "UniProtKB:Q15722",
  "gene_name": "Leukotriene B4 receptor 1",
  "term_label": "G protein-coupled peptide receptor activity"
}